{
  "gene_name": "Aldehyde dehydrogenase family 3 member B1",
  "gene": "UniProtKB:P43353",
  "term_label": "aldehyde dehydrogenase (NAD+) activity",
  "term_id": "GO:0004029",
  "gene_symbol": "ALDH3B1"
}